cell migration involved in vasculogenesis [GO:0035441] (biological process) Definition: The orderly movement of a cell from one site to another that will contribute to the differentiation of an endothelial cell that will form de novo blood vessels and tubes. Sources: GOC:dgh Relationships: is a type of cell migration [GO:0016477]; is part of GO:0001570 Subtypes: cell migration involved in coronary vasculogenesis [GO:0060980]